{
  "term_id": "GO:0048167",
  "gene_name": "Eukaryotic translation initiation factor 4E-binding protein 2",
  "gene_symbol": "EIF4EBP2",
  "term_label": "regulation of synaptic plasticity",
  "gene": "UniProtKB:Q13542"
}